{
  "term_id": "GO:0005615",
  "gene_symbol": "HPR",
  "term_label": "extracellular space",
  "gene_name": "Haptoglobin-related protein",
  "gene": "UniProtKB:P00739"
}